cardiac left ventricle morphogenesis [GO:0003214] (biological process) Relationships: is a type of cardiac ventricle morphogenesis [GO:0003208] Sources: GOC:mtg_heart Definition: The process in which the left cardiac ventricle is generated and organized.